{
  "gene": "UniProtKB:P60709",
  "gene_symbol": "ACTB",
  "term_id": "GO:0030424",
  "gene_name": "Actin, cytoplasmic 1",
  "term_label": "axon"
}